{
  "term_id": "GO:0019856",
  "gene_symbol": "CTPS2",
  "gene_name": "CTP synthase 2",
  "gene": "UniProtKB:Q9NRF8",
  "term_label": "pyrimidine nucleobase biosynthetic process"
}